{
  "gene_name": "Fibroblast growth factor 8",
  "term_label": "growth factor activity",
  "gene": "UniProtKB:P55075",
  "term_id": "GO:0008083",
  "gene_symbol": "FGF8"
}